{
  "gene_name": "Axin-2",
  "gene_symbol": "AXIN2",
  "term_id": "GO:0008013",
  "term_label": "beta-catenin binding",
  "gene": "UniProtKB:Q9Y2T1"
}